{
  "gene_symbol": "RNF19B",
  "term_id": "GO:0005737",
  "gene": "UniProtKB:Q6ZMZ0",
  "gene_name": "E3 ubiquitin-protein ligase RNF19B",
  "term_label": "cytoplasm"
}